type 2 galanin receptor binding [GO:0031765] (molecular function) Also known as: type 2 galanin receptor ligand Sources: GOC:mah, GOC:nln Definition: Binding to a type 2 galanin receptor. Relationships: is_a galanin receptor binding [GO:0031763]